{
  "gene_name": "Forkhead box protein D4-like 5",
  "gene_symbol": "FOXD4L5",
  "term_id": "GO:0000981",
  "term_label": "DNA-binding transcription factor activity, RNA polymerase II-specific",
  "gene": "UniProtKB:Q5VV16"
}